{
  "gene": "UniProtKB:Q12959",
  "term_label": "receptor clustering",
  "gene_symbol": "DLG1",
  "gene_name": "Disks large homolog 1",
  "term_id": "GO:0043113"
}